{
  "gene_symbol": "USP50",
  "term_id": "GO:0030496",
  "term_label": "midbody",
  "gene_name": "Inactive ubiquitin carboxyl-terminal hydrolase 50",
  "gene": "UniProtKB:Q70EL3"
}